 [go#goslim:virus] Note: GO subset for viruses